{
  "gene_name": "Guanine nucleotide-binding protein G(o) subunit alpha",
  "term_label": "adenylate cyclase-modulating G protein-coupled receptor signaling pathway",
  "gene_symbol": "GNAO1",
  "term_id": "GO:0007188",
  "gene": "UniProtKB:P09471"
}